1-phosphatidylinositol 4-kinase activity [GO:0004430] (molecular function) Also known as: PI kinase activity, phosphatidylinositol kinase (phosphorylating) activity, phosphatidylinositol kinase activity, PI 4-kinase activity, PI4-kinase activity, PI4K, PI4K-alpha activity, PtdIns-4-kinase activity, phosphatidylinositol 4-kinase activity, type II phosphatidylinositol kinase activity Definition: Catalysis of the reaction: a 1-phosphatidyl-1D-myo-inositol + ATP = a 1-phosphatidyl-1D-myo-inositol 4-phosphate + ADP + H+. Sources: EC:2.7.1.67, RHEA:19877 Regulation: positively regulated by 1-phosphatidylinositol 4-kinase activator activity [GO:0098744] Relationships: is a type of phosphatidylinositol kinase activity [GO:0052742]